identical protein binding [GO:0042802] (molecular function) Sources: GOC:jl Also known as: isoform-specific homophilic binding, protein homopolymerization Definition: Binding to an identical protein or proteins. Subtypes: GO:0042803 Relationships: is a type of protein binding [GO:0005515]